{
  "term_id": "GO:1990904",
  "gene_name": "RNA-binding motif, single-stranded-interacting protein 3",
  "gene": "UniProtKB:Q6XE24",
  "term_label": "ribonucleoprotein complex",
  "gene_symbol": "RBMS3"
}